{
  "gene_name": "Large ribosomal subunit protein mL55",
  "gene": "UniProtKB:Q7Z7F7",
  "gene_symbol": "MRPL55",
  "term_id": "GO:0006412",
  "term_label": "translation"
}